{
  "term_label": "Unknown molecular function",
  "term_id": "UNKNOWN:0001",
  "gene_name": "Uncharacterized protein",
  "gene": "UniProtKB:A0A0G2JND7",
  "gene_symbol": "A0A0G2JND7"
}